{
  "gene_name": "E3 ubiquitin-protein ligase PDZRN3",
  "gene": "UniProtKB:Q9UPQ7",
  "term_id": "GO:0007528",
  "term_label": "neuromuscular junction development",
  "gene_symbol": "PDZRN3"
}